{
  "gene": "UniProtKB:Q96FJ0",
  "gene_symbol": "STAMBPL1",
  "term_id": "GO:1904263",
  "term_label": "positive regulation of TORC1 signaling",
  "gene_name": "AMSH-like protease"
}